{
  "term_label": "RNA polymerase II cis-regulatory region sequence-specific DNA binding",
  "gene_name": "Zinc finger protein 581",
  "term_id": "GO:0000978",
  "gene_symbol": "ZNF581",
  "gene": "UniProtKB:Q9P0T4"
}